{
  "gene_name": "Estrogen-related receptor gamma",
  "gene_symbol": "ESRRG",
  "term_label": "nuclear receptor activity",
  "term_id": "GO:0004879",
  "gene": "UniProtKB:P62508"
}